CTP binding [GO:0002135] (MF) Relationships: is_a pyrimidine ribonucleotide binding [GO:0032557]; is a type of anion binding [GO:0043168] Sources: GOC:hjd, ISBN:0124020607 Definition: Binding to CTP, cytidine 5'-triphosphate.